{
  "term_id": "GO:0071949",
  "gene_name": "Proline dehydrogenase 1, mitochondrial",
  "gene": "UniProtKB:O43272",
  "gene_symbol": "PRODH",
  "term_label": "FAD binding"
}